regulation of CD4-positive, alpha-beta T cell proliferation [GO:2000561] (biological process) Subtypes: negative regulation of CD4-positive, alpha-beta T cell proliferation [GO:2000562], positive regulation of CD4-positive, alpha-beta T cell proliferation [GO:2000563] Definition: Any process that modulates the frequency, rate or extent of CD4-positive, alpha-beta T cell proliferation. Relationships: is a type of regulation of alpha-beta T cell proliferation [GO:0046640]; is a type of regulation of CD4-positive, alpha-beta T cell activation [GO:2000514]; regulates GO:0035739 Sources: GOC:obol